bile acid catabolic process [GO:0030573] (biological process) Relationships: is a type of bile acid metabolic process [GO:0008206]; is a type of monocarboxylic acid catabolic process [GO:0072329] Also known as: bile acid breakdown, bile acid catabolism, bile acid degradation, bile acid 7alpha-dehydroxylation pathway, cholate catabolic process Sources: GOC:go_curators Definition: The chemical reactions and pathways resulting in the breakdown of bile acids, any of a group of steroid carboxylic acids occurring in bile.